{
  "term_id": "GO:0061630",
  "gene": "UniProtKB:Q6ZVX7",
  "gene_symbol": "NCCRP1",
  "gene_name": "F-box only protein 50",
  "term_label": "ubiquitin protein ligase activity"
}